{
  "term_label": "regulation of transcription by RNA polymerase II",
  "gene_name": "Zinc finger and SCAN domain-containing protein 21",
  "term_id": "GO:0006357",
  "gene": "UniProtKB:Q9Y5A6",
  "gene_symbol": "ZSCAN21"
}